{
  "gene_symbol": "DNAJC9",
  "term_label": "nucleus",
  "term_id": "GO:0005634",
  "gene_name": "DnaJ homolog subfamily C member 9",
  "gene": "UniProtKB:Q8WXX5"
}